{
  "term_label": "extracellular matrix",
  "gene": "UniProtKB:Q8TE58",
  "gene_symbol": "ADAMTS15",
  "term_id": "GO:0031012",
  "gene_name": "A disintegrin and metalloproteinase with thrombospondin motifs 15"
}